negative regulation of growth hormone receptor signaling pathway [GO:0060400] (biological process) Definition: Any process that decreases the rate, frequency or extent of the growth hormone receptor signaling pathway. The growth hormone receptor signaling pathway is the series of molecular signals generated as a consequence of growth hormone receptor binding to its physiological ligand. Sources: GOC:dph Also known as: negative regulation of growth hormone receptor signalling pathway Relationships: is a type of negative regulation of signal transduction [GO:0009968]; is a type of regulation of growth hormone receptor signaling pathway [GO:0060398]; negatively regulates GO:0060396